{
  "gene_symbol": "P4HA3",
  "gene_name": "Prolyl 4-hydroxylase subunit alpha-3",
  "term_id": "GO:0004656",
  "term_label": "procollagen-proline 4-dioxygenase activity",
  "gene": "UniProtKB:Q7Z4N8"
}